regulation of L-glutamate import across plasma membrane [GO:0002036] (biological process) Relationships: is a type of regulation of amino acid import across plasma membrane [GO:0010958]; is_a regulation of organic acid transport [GO:0032890]; regulates L-glutamate import across plasma membrane [GO:0098712] Sources: GOC:TermGenie Definition: Any process that modulates the frequency, rate or extent of L-glutamate import into a cell. Also known as: regulation of L-glutamate import, regulation of L-glutamate transport, regulation of L-glutamate uptake Subtypes: GO:0002037, GO:0002038, regulation of glutamate uptake involved in transmission of nerve impulse [GO:0051946]